cellular response to copper ion [GO:0071280] (biological process) Definition: Any process that results in a change in state or activity of a cell (in terms of movement, secretion, enzyme production, gene expression, etc.) as a result of a copper ion stimulus. Sources: GOC:mah Also known as: cellular response to copper Relationships: is a type of response to copper ion [GO:0046688]; is a type of cellular response to metal ion [GO:0071248]